establishment or maintenance of cell polarity regulating cell shape [GO:0071963] (biological process) Sources: GOC:mah Relationships: is a type of establishment or maintenance of cell polarity [GO:0007163]; is_a regulation of cell shape [GO:0008360] Subtypes: GO:0061246, GO:0061340, establishment of cell polarity regulating cell shape [GO:0071964] Regulation: RO_0002211 by regulation of establishment or maintenance of cell polarity regulating cell shape [GO:2000769]; negatively regulated by GO:2000770; positively regulated by GO:2000771 Definition: Any cellular process that results in the specification, formation or maintenance of a polarized intracellular organization or cell growth patterns that regulate the shape of a cell.